{
  "gene_symbol": "KRT36",
  "term_id": "GO:0030855",
  "gene_name": "Keratin, type I cuticular Ha6",
  "gene": "UniProtKB:O76013",
  "term_label": "epithelial cell differentiation"
}